{
  "gene": "UniProtKB:P08173",
  "term_label": "G protein-coupled receptor signaling pathway, coupled to cyclic nucleotide second messenger",
  "gene_name": "Muscarinic acetylcholine receptor M4",
  "term_id": "GO:0007187",
  "gene_symbol": "CHRM4"
}